{
  "gene_symbol": "SF1",
  "term_label": "nucleus",
  "gene_name": "Splicing factor 1",
  "gene": "UniProtKB:Q15637",
  "term_id": "GO:0005634"
}